{
  "gene_symbol": "OR1L8",
  "term_id": "GO:0005886",
  "gene_name": "Olfactory receptor 1L8",
  "gene": "UniProtKB:Q8NGR8",
  "term_label": "plasma membrane"
}